{
  "term_label": "glutathione transferase activity",
  "term_id": "GO:0004364",
  "gene_name": "Glutathione S-transferase A1",
  "gene_symbol": "GSTA1",
  "gene": "UniProtKB:P08263"
}